regulation of peptide transport [GO:0090087] (BP) Sources: GOC:dph, GOC:tb Relationships: is a type of regulation of transport [GO:0051049]; regulates peptide transport [GO:0015833] Subtypes: regulation of peptide secretion [GO:0002791], regulation of oligopeptide transport [GO:0090088], GO:1901039 Definition: Any process that modulates the frequency, rate or extent of the directed movement of peptides, compounds of two or more amino acids where the alpha carboxyl group of one is bound to the alpha amino group of another, into, out of or within a cell, or between cells, by means of some agent such as a transporter or pore.